{
  "gene": "UniProtKB:A0A096LNW5",
  "term_id": "UNKNOWN:0003",
  "term_label": "Unknown cellular component",
  "gene_symbol": "NOTCH2NLR",
  "gene_name": "Notch homolog 2 N-terminal-like protein R"
}